{
  "gene": "UniProtKB:Q9BVA6",
  "gene_name": "Protein adenylyltransferase FICD",
  "term_label": "endoplasmic reticulum",
  "term_id": "GO:0005783",
  "gene_symbol": "FICD"
}